positive regulation of formation of symbiont germ tube hook structure for appressorium development [GO:0075031] (biological process) Definition: Any process that activates, maintains or increases the frequency, rate or extent of symbiont germ tube hook structure formation. Sources: GOC:pamgo_curators Also known as: positive regulation of formation of symbiont germ tube hook structure on or near host, positive regulation of germ tube tip of symbiont on or near the exterior of host, positive regulation of symbiont germ tube hook structure formation on or near host Relationships: is a type of positive regulation of developmental process [GO:0051094]; is a type of GO:0075030; positively regulates formation of appressorium germ tube hook structure [GO:0075029]